positive regulation of heart induction [GO:1901321] (biological process) Relationships: is a type of regulation of heart induction [GO:0090381]; is_a positive regulation of animal organ morphogenesis [GO:0110110]; positively regulates heart induction [GO:0003129] Also known as: up regulation of heart induction, up-regulation of heart induction, upregulation of heart induction, activation of heart induction Definition: Any process that activates or increases the frequency, rate or extent of heart induction. Sources: GOC:TermGenie